{
  "gene_name": "Zinc finger-containing ubiquitin peptidase 1",
  "gene": "UniProtKB:Q96AP4",
  "term_label": "nucleus",
  "gene_symbol": "ZUP1",
  "term_id": "GO:0005634"
}